{
  "term_label": "tRNA-specific adenosine-34 deaminase activity",
  "gene_name": "tRNA-specific adenosine deaminase 2",
  "gene": "UniProtKB:Q7Z6V5",
  "gene_symbol": "ADAT2",
  "term_id": "GO:0052717"
}